{
  "gene_symbol": "NPW",
  "gene_name": "Neuropeptide W",
  "term_id": "GO:0007186",
  "term_label": "G protein-coupled receptor signaling pathway",
  "gene": "UniProtKB:Q8N729"
}